beta-glucan catabolic process [GO:0051275] (biological process) Sources: GOC:ai Also known as: beta-glucan breakdown, beta-glucan catabolism, beta-glucan degradation Subtypes: (1->3)-beta-D-glucan catabolic process [GO:0006076], (1->6)-beta-D-glucan catabolic process [GO:0006079], cellulose catabolic process [GO:0030245] Definition: The chemical reactions and pathways resulting in the breakdown of beta-glucans. Relationships: is a type of GO:0009251; is a type of beta-glucan metabolic process [GO:0051273]